cellular response to 3,3',4,4',5-pentachlorobiphenyl [GO:1904611] (biological process) Also known as: cellular response to PCB 126 Relationships: is_a GO:0070887; is a type of response to 3,3',4,4',5-pentachlorobiphenyl [GO:1904610] Definition: Any process that results in a change in state or activity of a cell (in terms of movement, secretion, enzyme production, gene expression, etc.) as a result of a 3,3',4,4',5-pentachlorobiphenyl stimulus. References: PMID:23196670 Sources: GOC:TermGenie, GO_REF:0000071